{
  "gene_name": "Nucleolar protein 16",
  "gene_symbol": "NOP16",
  "term_label": "nucleolus",
  "term_id": "GO:0005730",
  "gene": "UniProtKB:Q9Y3C1"
}